{
  "gene_symbol": "OBSL1",
  "term_label": "positive regulation of dendrite morphogenesis",
  "gene": "UniProtKB:O75147",
  "gene_name": "Obscurin-like protein 1",
  "term_id": "GO:0050775"
}